protein import [GO:0017038] (biological process) Also known as: protein uptake Subtypes: GO:0045038 Relationships: is a type of protein transport [GO:0015031] Regulation: regulated by regulation of protein import [GO:1904589]; negatively regulated by negative regulation of protein import [GO:1904590]; positively regulated by positive regulation of protein import [GO:1904591] Sources: GOC:ai Definition: The targeting and directed movement of proteins into a cell or organelle. Not all import involves an initial targeting event.